{
  "gene_name": "Small ribosomal subunit protein uS14",
  "gene_symbol": "RPS29",
  "term_label": "zinc ion binding",
  "term_id": "GO:0008270",
  "gene": "UniProtKB:P62273"
}